{
  "gene": "UniProtKB:P62244",
  "gene_symbol": "RPS15A",
  "term_label": "cytosolic small ribosomal subunit",
  "term_id": "GO:0022627",
  "gene_name": "Small ribosomal subunit protein uS8"
}